{
  "gene_name": "Phosphatidylinositol-binding clathrin assembly protein",
  "gene_symbol": "PICALM",
  "term_label": "extrinsic component of presynaptic endocytic zone membrane",
  "gene": "UniProtKB:Q13492",
  "term_id": "GO:0098894"
}